{
  "gene_symbol": "PEAK3",
  "term_id": "GO:0004672",
  "gene": "UniProtKB:Q6ZS72",
  "term_label": "protein kinase activity",
  "gene_name": "Protein PEAK3"
}